galactolipid galactosyltransferase activity [GO:0046480] (molecular function) Definition: Catalysis of the reaction: 2 mono-beta-D-galactosyldiacylglycerol = alpha-D-galactosyl-beta-D-galactosyldiacylglycerol + 1,2-diacylglycerol. Sources: EC:2.4.1.184 Relationships: is a type of GO:0008378 Also known as: DGDG synthase activity, digalactosyldiacylglycerol synthase activity, galactolipid:galactolipid galactosyltransferase activity, 3-(beta-D-galactosyl)-1,2-diacyl-sn-glycerol:mono-3-(beta-D-galactosyl)-1,2-diacyl-sn-glycerol beta-D-galactosyltransferase activity, GGGT activity, galactolipid-galactolipid galactosyltransferase activity, interlipid galactosyltransferase activity